circadian sleep/wake cycle, sleep [GO:0050802] (biological process) Definition: The part of the circadian sleep/wake cycle where the organism is asleep. Sources: GOC:ai Regulation: RO_0002212 by negative regulation of circadian sleep/wake cycle, sleep [GO:0042321]; regulated by GO:0045187; positively regulated by GO:0045938 Relationships: is a type of circadian sleep/wake cycle process [GO:0022410]; is_a sleep [GO:0030431]